{
  "gene_symbol": "RIMS2",
  "term_label": "synaptic vesicle priming",
  "gene_name": "Regulating synaptic membrane exocytosis protein 2",
  "gene": "UniProtKB:Q9UQ26",
  "term_id": "GO:0016082"
}